{
  "gene_name": "E3 ubiquitin-protein ligase SIAH1",
  "term_id": "GO:0005737",
  "gene": "UniProtKB:Q8IUQ4",
  "gene_symbol": "SIAH1",
  "term_label": "cytoplasm"
}